{
  "gene_symbol": "CDK1",
  "gene_name": "Cyclin-dependent kinase 1",
  "term_label": "cyclin-dependent protein kinase holoenzyme complex",
  "term_id": "GO:0000307",
  "gene": "UniProtKB:P06493"
}